{
  "gene_symbol": "PNAS-138",
  "term_id": "UNKNOWN:0003",
  "gene": "UniProtKB:Q9BZS9",
  "gene_name": "Putative uncharacterized protein PNAS-138",
  "term_label": "Unknown cellular component"
}